{
  "gene": "UniProtKB:Q5T160",
  "term_id": "GO:0005739",
  "term_label": "mitochondrion",
  "gene_symbol": "RARS2",
  "gene_name": "Probable arginine--tRNA ligase, mitochondrial"
}